regulation of replication fork arrest at rDNA repeats [GO:1902681] (biological process) Relationships: is a type of regulation of chromosome organization [GO:0033044]; is a type of GO:0090329; regulates replication fork arrest at rDNA repeats [GO:0031582] Also known as: regulation of replication fork arrest at ribosomal DNA repeats, regulation of replication fork blocking at rDNA repeats Definition: Any process that modulates the frequency, rate or extent of replication fork arrest at rDNA repeats. References: PMID:23260662 Sources: GOC:TermGenie, GO_REF:0000058